{
  "gene_name": "Protein phosphatase 1 regulatory subunit 32",
  "gene": "UniProtKB:Q7Z5V6",
  "term_id": "UNKNOWN:0002",
  "gene_symbol": "PPP1R32",
  "term_label": "Unknown biological process"
}